{
  "gene": "UniProtKB:Q9BW04",
  "term_id": "UNKNOWN:0002",
  "gene_symbol": "SARG",
  "term_label": "Unknown biological process",
  "gene_name": "Specifically androgen-regulated gene protein"
}